{
  "gene_name": "Uncharacterized protein",
  "gene": "UniProtKB:A0A2R9YJI8",
  "term_label": "Unknown molecular function",
  "gene_symbol": "A0A2R9YJI8",
  "term_id": "UNKNOWN:0001"
}